positive regulation of skeletal muscle fiber differentiation [GO:1902811] (biological process) Subtypes: GO:2001037 Relationships: is a type of positive regulation of myotube differentiation [GO:0010831]; is a type of regulation of skeletal muscle fiber differentiation [GO:1902809]; is a type of positive regulation of skeletal muscle cell differentiation [GO:2001016]; positively regulates skeletal muscle fiber differentiation [GO:0098528] References: PMID:17879321 Sources: GOC:TermGenie, GOC:mr, GO_REF:0000058 Also known as: up regulation of skeletal muscle fiber differentiation, up-regulation of skeletal muscle fiber differentiation, upregulation of skeletal muscle fiber differentiation, activation of skeletal muscle fiber differentiation Definition: Any process that activates or increases the frequency, rate or extent of skeletal muscle fiber differentiation.